{
  "term_id": "GO:0000146",
  "gene": "UniProtKB:P13533",
  "gene_symbol": "MYH6",
  "gene_name": "Myosin-6",
  "term_label": "microfilament motor activity"
}